{
  "gene_symbol": "CPLX2",
  "term_id": "GO:0031630",
  "gene_name": "Complexin-2",
  "term_label": "regulation of synaptic vesicle fusion to presynaptic active zone membrane",
  "gene": "UniProtKB:Q6PUV4"
}